{
  "gene_symbol": "CDC5L",
  "gene_name": "Cell division cycle 5-like protein",
  "gene": "UniProtKB:Q99459",
  "term_id": "GO:0000398",
  "term_label": "mRNA splicing, via spliceosome"
}